{
  "gene": "UniProtKB:Q9BRQ6",
  "gene_name": "MICOS complex subunit MIC25",
  "term_id": "UNKNOWN:0001",
  "term_label": "Unknown molecular function",
  "gene_symbol": "CHCHD6"
}